{
  "gene_name": "Olfactory receptor 13C9",
  "term_id": "GO:0050911",
  "gene": "UniProtKB:Q8NGT0",
  "gene_symbol": "OR13C9",
  "term_label": "detection of chemical stimulus involved in sensory perception of smell"
}